{
  "term_id": "GO:0005737",
  "term_label": "cytoplasm",
  "gene": "UniProtKB:Q9NUK0",
  "gene_symbol": "MBNL3",
  "gene_name": "Muscleblind-like protein 3"
}